{
  "term_label": "transmembrane transporter activity",
  "gene_symbol": "SLC25A47",
  "term_id": "GO:0022857",
  "gene_name": "Solute carrier family 25 member 47",
  "gene": "UniProtKB:Q6Q0C1"
}